{
  "gene": "UniProtKB:P28356",
  "gene_symbol": "HOXD9",
  "term_id": "GO:0009952",
  "term_label": "anterior/posterior pattern specification",
  "gene_name": "Homeobox protein Hox-D9"
}